{
  "gene": "UniProtKB:A0A1B0GTD5",
  "gene_symbol": "SPMIP11",
  "term_id": "UNKNOWN:0001",
  "term_label": "Unknown molecular function",
  "gene_name": "Testis-expressed protein 49"
}